cellular response to glutathione [GO:0072753] (biological process) Sources: GOC:mah Relationships: is a type of response to glutathione [GO:1901370]; is a type of cellular response to nitrogen compound [GO:1901699]; is a type of cellular response to oxygen-containing compound [GO:1901701] Definition: Any process that results in a change in state or activity of a cell (in terms of movement, secretion, enzyme production, gene expression, etc.) as a result of a glutathione stimulus.